{
  "gene_symbol": "CD34",
  "gene_name": "Hematopoietic progenitor cell antigen CD34",
  "gene": "UniProtKB:P28906",
  "term_label": "Unknown molecular function",
  "term_id": "UNKNOWN:0001"
}